{
  "gene": "UniProtKB:O60701",
  "term_label": "glycosaminoglycan biosynthetic process",
  "gene_symbol": "UGDH",
  "term_id": "GO:0006024",
  "gene_name": "UDP-glucose 6-dehydrogenase"
}